{
  "term_label": "mitochondrion",
  "gene_name": "Pyruvate carboxylase, mitochondrial",
  "gene": "UniProtKB:P11498",
  "term_id": "GO:0005739",
  "gene_symbol": "PC"
}